{
  "term_id": "UNKNOWN:0002",
  "term_label": "Unknown biological process",
  "gene_name": "Small cysteine and glycine repeat-containing protein 6",
  "gene_symbol": "SCYGR6",
  "gene": "UniProtKB:A0A286YF77"
}